{
  "gene": "UniProtKB:Q9ULM6",
  "gene_symbol": "CNOT6",
  "term_id": "UNKNOWN:0002",
  "gene_name": "CCR4-NOT transcription complex subunit 6",
  "term_label": "Unknown biological process"
}